{
  "term_id": "GO:0003924",
  "term_label": "GTPase activity",
  "gene_symbol": "SRP54",
  "gene": "UniProtKB:P61011",
  "gene_name": "Signal recognition particle subunit SRP54"
}